{
  "term_label": "Unknown cellular component",
  "gene_name": "Large ribosomal subunit protein uL4m",
  "gene": "UniProtKB:Q9BYD3",
  "gene_symbol": "MRPL4",
  "term_id": "UNKNOWN:0003"
}